{
  "term_label": "1-phosphatidylinositol-4-phosphate 5-kinase activity",
  "term_id": "GO:0016308",
  "gene": "UniProtKB:A2A3N6",
  "gene_name": "Putative PIP5K1A and PSMD4-like protein",
  "gene_symbol": "PIPSL"
}